Nrd1 complex [GO:0035649] (cellular component) References: PMID:10655211, PMID:16427013, PMID:21084293 Sources: GOC:jh Relationships: is a type of GO:0032991 Definition: A complex that functions in transcription termination of RNA polymerase II transcribed non-coding RNAs. This complex interacts with the carboxy-terminal domain (CTD) of PolII and the terminator sequences in the nascent RNA transcript. In yeast this complex consists of Nrd1p, Nab3p, and Sen1p.